{
  "term_id": "GO:0050911",
  "term_label": "detection of chemical stimulus involved in sensory perception of smell",
  "gene_name": "Olfactory receptor 10H2",
  "gene_symbol": "OR10H2",
  "gene": "UniProtKB:O60403"
}